{
  "gene_name": "Secretoglobin family 1C member 2",
  "gene_symbol": "SCGB1C2",
  "term_id": "UNKNOWN:0003",
  "term_label": "Unknown cellular component",
  "gene": "UniProtKB:P0DMR2"
}